{
  "term_id": "GO:0005886",
  "term_label": "plasma membrane",
  "gene": "UniProtKB:Q4KMQ2",
  "gene_symbol": "ANO6",
  "gene_name": "Anoctamin-6"
}